{
  "gene_name": "Fibulin-7",
  "term_id": "GO:0005615",
  "term_label": "extracellular space",
  "gene": "UniProtKB:Q53RD9",
  "gene_symbol": "FBLN7"
}